negative regulation of postsynaptic membrane organization [GO:1901627] (biological process) Definition: Any process that stops, prevents or reduces the frequency, rate or extent of postsynaptic membrane organization. References: PMID:22426000 Sources: GOC:TermGenie Also known as: down regulation of postsynaptic membrane organisation, down regulation of postsynaptic membrane organization, down-regulation of postsynaptic membrane organisation, down-regulation of postsynaptic membrane organization, downregulation of postsynaptic membrane organisation, downregulation of postsynaptic membrane organization, negative regulation of post-synaptic membrane organization, negative regulation of postsynaptic membrane organisation, inhibition of postsynaptic membrane organisation, inhibition of postsynaptic membrane organization Relationships: is a type of regulation of postsynaptic membrane organization [GO:1901626]; is a type of negative regulation of synapse organization [GO:1905809]; negatively regulates postsynaptic membrane organization [GO:0001941] Subtypes: negative regulation of AMPA glutamate receptor clustering [GO:1904718]